{
  "gene_name": "GTP-binding protein Di-Ras1",
  "term_label": "small GTPase-mediated signal transduction",
  "gene": "UniProtKB:O95057",
  "gene_symbol": "DIRAS1",
  "term_id": "GO:0007264"
}